dorsal lateral ganglionic eminence cell proliferation [GO:0022019] (BP) Definition: The multiplication or reproduction of dorsal lateral ganglionic eminence cells, resulting in the expansion of the cell population. Sources: GOC:cls, GOC:dgh, GOC:dph, GOC:jid, GO_REF:0000021 Relationships: is a type of GO:0022012; is part of GO:0022018